neutral amino acid transport [GO:0015804] (BP) Subtypes: beta-alanine transport [GO:0001762], GO:0006867, GO:0006868, L-cystine transport [GO:0015811], glycine transport [GO:0015816], isoleucine transport [GO:0015818], GO:0015820, proline transport [GO:0015824], GO:0015826, GO:0015829, alanine transport [GO:0032328], serine transport [GO:0032329], neutral amino acid transmembrane export from vacuole [GO:0034489], GO:0034491, GO:0042883, homoserine transport [GO:0042968] Sources: GOC:ai Definition: The directed movement of neutral amino acids, amino acids with no net charge, into, out of or within a cell, or between cells, by means of some agent such as a transporter or pore. Relationships: is a type of amino acid transport [GO:0006865]